{
  "term_label": "nucleus",
  "gene_symbol": "APOBEC3H",
  "term_id": "GO:0005634",
  "gene_name": "DNA dC-dU-editing enzyme APOBEC-3H",
  "gene": "UniProtKB:Q6NTF7"
}